{
  "gene": "UniProtKB:Q5FWF6",
  "term_id": "GO:0000978",
  "gene_name": "Zinc finger protein 789",
  "term_label": "RNA polymerase II cis-regulatory region sequence-specific DNA binding",
  "gene_symbol": "ZNF789"
}